{
  "gene": "UniProtKB:Q8IVF2",
  "term_label": "cytoplasm",
  "gene_symbol": "AHNAK2",
  "gene_name": "Protein AHNAK2",
  "term_id": "GO:0005737"
}